{
  "gene_name": "Cytochrome P450 2E1",
  "term_id": "GO:0020037",
  "gene_symbol": "CYP2E1",
  "term_label": "heme binding",
  "gene": "UniProtKB:P05181"
}